{
  "gene_name": "L-seryl-tRNA(Sec) kinase",
  "term_id": "UNKNOWN:0002",
  "gene": "UniProtKB:Q8IV42",
  "gene_symbol": "PSTK",
  "term_label": "Unknown biological process"
}